tertiary alcohol biosynthetic process [GO:1902645] (biological process) Also known as: tertiary alcohol anabolism, tertiary alcohol biosynthesis, tertiary alcohol formation, tertiary alcohol synthesis Subtypes: abscisic acid biosynthetic process [GO:0009688], GO:0019289, cortisol biosynthetic process [GO:0034651], tetracycline biosynthetic process [GO:0043644], viridicatumtoxin biosynthetic process [GO:0140872], paxilline biosynthetic process [GO:0140873], paraherquonin biosynthetic process [GO:0140874], asperfuranone biosynthetic process [GO:1900554], GO:1900985, GO:1901106, GO:1902050, GO:1902246 References: PMID:11288200 Sources: GOC:TermGenie, GOC:mengo_curators, GO_REF:0000068 Definition: The chemical reactions and pathways resulting in the formation of tertiary alcohol. Relationships: is_a alcohol biosynthetic process [GO:0046165]; is a type of GO:1902644